{
  "gene": "UniProtKB:Q96JK2",
  "gene_name": "DDB1- and CUL4-associated factor 5",
  "term_id": "UNKNOWN:0001",
  "gene_symbol": "DCAF5",
  "term_label": "Unknown molecular function"
}